{
  "term_id": "GO:0031410",
  "term_label": "cytoplasmic vesicle",
  "gene_name": "Porimin",
  "gene": "UniProtKB:Q8N131",
  "gene_symbol": "TMEM123"
}